{
  "gene_symbol": "ESYT1",
  "term_label": "phosphatidylinositol binding",
  "gene": "UniProtKB:Q9BSJ8",
  "term_id": "GO:0035091",
  "gene_name": "Extended synaptotagmin-1"
}